{
  "gene": "UniProtKB:Q8N2K0",
  "gene_name": "Lysophosphatidylserine lipase ABHD12",
  "term_label": "monoacylglycerol catabolic process",
  "gene_symbol": "ABHD12",
  "term_id": "GO:0052651"
}